{
  "term_label": "DNA-binding transcription factor activity, RNA polymerase II-specific",
  "term_id": "GO:0000981",
  "gene_symbol": "OLIG2",
  "gene_name": "Oligodendrocyte transcription factor 2",
  "gene": "UniProtKB:Q13516"
}